right ventricular trabecular myocardium morphogenesis [GO:0003227] (biological process) Relationships: is a type of GO:0003221; is_a ventricular trabecula myocardium morphogenesis [GO:0003222] Definition: The process in which the anatomical structures of the right ventricular myocardium are generated and organized. Sources: GOC:mtg_heart